positive regulation of amyloid-beta clearance [GO:1900223] (BP) Relationships: is a type of positive regulation of multicellular organismal process [GO:0051240]; is a type of GO:1900221; positively regulates amyloid-beta clearance [GO:0097242] Sources: GOC:BHF, GOC:TermGenie Also known as: positive regulation of beta-amyloid clearance, up regulation of beta-amyloid clearance, up-regulation of beta-amyloid clearance, upregulation of beta-amyloid clearance, activation of beta-amyloid clearance Definition: Any process that activates or increases the frequency, rate or extent of amyloid-beta clearance.